{
  "gene_name": "Echinoderm microtubule-associated protein-like 4",
  "gene_symbol": "EML4",
  "gene": "UniProtKB:Q9HC35",
  "term_label": "microtubule cytoskeleton organization",
  "term_id": "GO:0000226"
}